glutamine N-phenylacetyltransferase activity [GO:0047947] (molecular function) Definition: Catalysis of the reaction: phenylacetyl-CoA + L-glutamine = CoA + alpha-N-phenylacetyl-L-glutamine. Sources: EC:2.3.1.14, MetaCyc:GLUTAMINE-N-PHENYLACETYLTRANSFERASE-RXN Relationships: is a type of acyltransferase activity, transferring groups other than amino-acyl groups [GO:0016747] Also known as: glutamine phenylacetyltransferase activity, phenylacetyl-CoA:L-glutamine N-acetyltransferase activity, phenylacetyl-CoA:L-glutamine alpha-N-phenylacetyltransferase activity